negative regulation of thiamine diphosphate biosynthetic process [GO:0070617] (biological process) Sources: GOC:mah Also known as: down regulation of thiamine diphosphate biosynthetic process, down-regulation of thiamine diphosphate biosynthetic process, downregulation of thiamine diphosphate biosynthetic process, negative regulation of thiamin diphosphate biosynthetic process, negative regulation of thiamine diphosphate anabolism, negative regulation of thiamine diphosphate biosynthesis, negative regulation of thiamine diphosphate formation, negative regulation of thiamine diphosphate synthesis, inhibition of thiamine diphosphate biosynthetic process Relationships: is a type of negative regulation of biosynthetic process [GO:0009890]; is a type of negative regulation of phosphate metabolic process [GO:0045936]; is a type of negative regulation of vitamin metabolic process [GO:0046137]; is_a regulation of thiamine diphosphate biosynthetic process [GO:0070616]; negatively regulates thiamine diphosphate biosynthetic process [GO:0009229] Definition: Any process that stops, prevents, or reduces the frequency, rate or extent of the chemical reactions and pathways resulting in the formation of thiamine diphosphate.